{
  "gene": "UniProtKB:Q8IZA0",
  "gene_symbol": "KIAA0319L",
  "term_id": "UNKNOWN:0001",
  "term_label": "Unknown molecular function",
  "gene_name": "Dyslexia-associated protein KIAA0319-like protein"
}